{
  "term_label": "plasma membrane",
  "gene_name": "Olfactory receptor 13C8",
  "gene": "UniProtKB:Q8NGS7",
  "gene_symbol": "OR13C8",
  "term_id": "GO:0005886"
}